apposition of dorsal and ventral imaginal disc-derived wing surfaces [GO:0007475] (biological process) Relationships: is a type of post-embryonic animal morphogenesis [GO:0009886]; is part of imaginal disc-derived wing margin morphogenesis [GO:0008587] Sources: GOC:bf, GOC:mtg_sensu Definition: The coming together of the dorsal and ventral surfaces of the imaginal disc-derived wing during the conversion of a folded single layered wing disc to a flat bilayered wing. Also known as: apposition of dorsal and ventral wing surfaces